{
  "gene": "UniProtKB:Q8IW40",
  "gene_symbol": "CCDC103",
  "term_id": "GO:0036159",
  "term_label": "inner dynein arm assembly",
  "gene_name": "Coiled-coil domain-containing protein 103"
}